{
  "gene_name": "Alpha-1,3_1,6-mannosyltransferase ALG2",
  "term_label": "alpha-1,3-mannosyltransferase activity",
  "gene": "UniProtKB:Q9H553",
  "term_id": "GO:0000033",
  "gene_symbol": "ALG2"
}